{
  "gene": "UniProtKB:P53675",
  "gene_symbol": "CLTCL1",
  "term_label": "clathrin-coated endocytic vesicle",
  "gene_name": "Clathrin heavy chain 2",
  "term_id": "GO:0045334"
}